{
  "gene_name": "Ras-related protein Rab-22A",
  "term_label": "intracellular protein transport",
  "gene_symbol": "RAB22A",
  "term_id": "GO:0006886",
  "gene": "UniProtKB:Q9UL26"
}